{
  "gene": "UniProtKB:Q8IZT6",
  "term_label": "Unknown cellular component",
  "term_id": "UNKNOWN:0003",
  "gene_name": "Abnormal spindle-like microcephaly-associated protein",
  "gene_symbol": "ASPM"
}